{
  "gene_name": "Steroidogenic factor 1",
  "gene": "UniProtKB:Q13285",
  "term_label": "RNA polymerase II cis-regulatory region sequence-specific DNA binding",
  "term_id": "GO:0000978",
  "gene_symbol": "NR5A1"
}